{
  "gene_name": "Large ribosomal subunit protein eL30",
  "term_label": "cytosolic large ribosomal subunit",
  "term_id": "GO:0022625",
  "gene": "UniProtKB:P62888",
  "gene_symbol": "RPL30"
}